prefoldin complex [GO:0016272] (cellular component) Definition: A multisubunit chaperone that is capable of delivering unfolded proteins to cytosolic chaperonin, which it acts as a cofactor for. In humans, the complex is a heterohexamer of two PFD-alpha and four PFD-beta type subunits. In Saccharomyces cerevisiae, it also acts in the nucleus to regulate the rate of elongation by RNA polymerase II via a direct effect on histone dynamics. References: PMID:17384227, PMID:24068951, PMID:9630229 Sources: GOC:jl Relationships: is a type of protein-containing complex [GO:0032991] Also known as: GIM complex